{
  "term_id": "GO:0005634",
  "gene_symbol": "TRMT10B",
  "gene": "UniProtKB:Q6PF06",
  "gene_name": "tRNA methyltransferase 10 homolog B",
  "term_label": "nucleus"
}